plant-type primary cell wall biogenesis [GO:0009833] (biological process) Definition: A cellular process that results in the biosynthesis of constituent macromolecules, assembly, and arrangement of constituent parts of cellulose and pectin-containing cell walls that form adjacent to the middle lamella following cell division and during cell expansion. An example of this is found in Arabidopsis thaliana. Also known as: primary cell wall anabolism, primary cell wall biosynthetic process, primary cell wall formation, primary cell wall synthesis, cellulose and pectin-containing primary cell wall biogenesis, primary cell wall biogenesis Sources: GOC:lr, GOC:mtg_sensu Relationships: is a type of plant-type cell wall biogenesis [GO:0009832]; is a type of mitotic cell cycle process [GO:1903047]; is part of GO:0000281